{
  "gene": "UniProtKB:Q9H8S5",
  "term_id": "GO:0005634",
  "gene_symbol": "CCNP",
  "gene_name": "Cyclin-P",
  "term_label": "nucleus"
}